benzoyl acetate-CoA thiolase activity [GO:0018711] (MF) Sources: UM-BBD_reactionID:r0243 Relationships: is a type of acyltransferase activity, transferring groups other than amino-acyl groups [GO:0016747] Definition: Catalysis of the reaction: benzoyl acetyl-CoA + CoA = acetyl-CoA + benzoyl-CoA.